{
  "gene_symbol": "PKP4",
  "term_label": "adherens junction",
  "gene": "UniProtKB:Q99569",
  "term_id": "GO:0005912",
  "gene_name": "Plakophilin-4"
}